{
  "gene": "UniProtKB:Q9P0M4",
  "term_id": "UNKNOWN:0003",
  "term_label": "Unknown cellular component",
  "gene_symbol": "IL17C",
  "gene_name": "Interleukin-17C"
}